{
  "gene_name": "Cytochrome P450 4F8",
  "gene": "UniProtKB:P98187",
  "term_id": "UNKNOWN:0003",
  "gene_symbol": "CYP4F8",
  "term_label": "Unknown cellular component"
}